{
  "gene": "UniProtKB:O43294",
  "gene_symbol": "TGFB1I1",
  "gene_name": "Transforming growth factor beta-1-induced transcript 1 protein",
  "term_label": "focal adhesion",
  "term_id": "GO:0005925"
}